methylgallate biosynthetic process [GO:0046277] (biological process) Definition: The chemical reactions and pathways resulting in the formation of methylgallate, trihydroxymethylbenzoate, the anion of methylgallic acid. Sources: GOC:ai Also known as: methylgallate anabolism, methylgallate biosynthesis, methylgallate formation, methylgallate synthesis Relationships: is a type of catechol-containing compound biosynthetic process [GO:0009713]; is a type of benzene-containing compound metabolic process [GO:0042537]; is a type of GO:0072330